{
  "gene": "UniProtKB:Q3LI60",
  "gene_symbol": "KRTAP20-3",
  "gene_name": "Keratin-associated protein 20-3",
  "term_id": "UNKNOWN:0003",
  "term_label": "Unknown cellular component"
}